{
  "term_id": "GO:0005634",
  "term_label": "nucleus",
  "gene_symbol": "CTNNB1",
  "gene_name": "Catenin beta-1",
  "gene": "UniProtKB:P35222"
}